{
  "term_id": "GO:0061630",
  "gene": "UniProtKB:Q8N7C7",
  "term_label": "ubiquitin protein ligase activity",
  "gene_name": "RING finger protein 148",
  "gene_symbol": "RNF148"
}